{
  "term_label": "nucleus",
  "gene": "UniProtKB:P40306",
  "gene_symbol": "PSMB10",
  "gene_name": "Proteasome subunit beta type-10",
  "term_id": "GO:0005634"
}